{
  "gene": "UniProtKB:P49407",
  "gene_symbol": "ARRB1",
  "term_label": "sensory perception",
  "term_id": "GO:0007600",
  "gene_name": "Beta-arrestin-1"
}